{
  "gene_symbol": "POU6F1",
  "gene": "UniProtKB:Q14863",
  "term_label": "RNA polymerase II cis-regulatory region sequence-specific DNA binding",
  "gene_name": "POU domain, class 6, transcription factor 1",
  "term_id": "GO:0000978"
}